negative regulation of antigen processing and presentation of peptide antigen via MHC class Ib [GO:0002596] (biological process) Sources: GOC:add Definition: Any process that stops, prevents, or reduces the frequency, rate, or extent of antigen processing and presentation of peptide antigen via MHC class Ib. Also known as: down regulation of antigen processing and presentation of peptide antigen via MHC class Ib, down-regulation of antigen processing and presentation of peptide antigen via MHC class Ib, downregulation of antigen processing and presentation of peptide antigen via MHC class Ib, negative regulation of peptide antigen processing and presentation via MHC class Ib, inhibition of antigen processing and presentation of peptide antigen via MHC class Ib Relationships: is a type of GO:0002584; is a type of negative regulation of antigen processing and presentation via MHC class Ib [GO:0002593]; is a type of regulation of antigen processing and presentation of peptide antigen via MHC class Ib [GO:0002595]; negatively regulates antigen processing and presentation of peptide antigen via MHC class Ib [GO:0002428]